glucose mediated signaling pathway [GO:0010255] (biological process) Regulation: regulated by GO:1902659; negatively regulated by GO:1902660; positively regulated by positive regulation of glucose mediated signaling pathway [GO:1902661] Sources: GOC:sm Also known as: glucose mediated signalling Relationships: is a type of hexose mediated signaling [GO:0009757]; is part of cellular response to glucose stimulus [GO:0071333] Definition: The process in which a change in the level of mono- and disaccharide glucose trigger the expression of genes controlling metabolic and developmental processes.